{
  "gene": "UniProtKB:Q96P47",
  "gene_name": "Arf-GAP with GTPase, ANK repeat and PH domain-containing protein 3",
  "gene_symbol": "AGAP3",
  "term_label": "GTPase activator activity",
  "term_id": "GO:0005096"
}